carbohydrate utilization [GO:0009758] (biological process) Sources: GOC:mah, GOC:mcc2, GOC:mlg Also known as: sugar utilization Definition: A series of processes that forms an integrated mechanism by which a cell or an organism detects the depletion of primary carbohydrate sources,usually glucose, and then activates genes to scavenge the last traces of the primary carbohydrate source and to transport and metabolize alternate carbohydrate sources. The utilization process begins when the cell or organism detects carbohydrate levels, includes the activation of genes whose products detect, transport or metabolize carbohydrates, and ends when the carbohydrate is incorporated into the cell or organism's metabolism. Regulation: RO_0002211 by GO:0043610 Relationships: is a type of GO:0031667; has part GO:0005975; has part carbohydrate transport [GO:0008643]